{
  "gene": "UniProtKB:P62314",
  "gene_name": "Small nuclear ribonucleoprotein Sm D1",
  "term_id": "GO:0005682",
  "term_label": "U5 snRNP",
  "gene_symbol": "SNRPD1"
}